{
  "gene": "UniProtKB:O76009",
  "gene_name": "Keratin, type I cuticular Ha3-I",
  "term_id": "GO:0045109",
  "gene_symbol": "KRT33A",
  "term_label": "intermediate filament organization"
}